{
  "term_label": "Unknown biological process",
  "gene": "UniProtKB:O00322",
  "gene_symbol": "UPK1A",
  "term_id": "UNKNOWN:0002",
  "gene_name": "Uroplakin-1a"
}